L-tyrosine-2-oxoglutarate transaminase activity [GO:0004838] (molecular function) Sources: RHEA:15093 Also known as: L-tyrosine aminotransferase activity, L-tyrosine transaminase activity, tyrosine aminotransferase activity, tyrosine transaminase activity, tyrosine-2-ketoglutarate aminotransferase activity, tyrosine-alpha-ketoglutarate aminotransferase activity, tyrosine-alpha-ketoglutarate transaminase activity, L-tyrosine:2-oxoglutarate aminotransferase activity, L-phenylalanine 2-oxoglutarate aminotransferase activity, TyrAT activity, glutamic phenylpyruvic aminotransferase activity, glutamic-hydroxyphenylpyruvic transaminase activity, phenylalanine aminotransferase activity, phenylalanine transaminase activity, phenylalanine-alpha-ketoglutarate transaminase activity, phenylpyruvate transaminase activity, phenylpyruvic acid transaminase activity Definition: Catalysis of the reaction: L-tyrosine + 2-oxoglutarate = 4-hydroxyphenylpyruvate + L-glutamate. Relationships: is a type of aromatic-amino-acid transaminase activity [GO:0008793]